negative regulation of timing of catagen [GO:0051796] (biological process) Relationships: is_a GO:0048817; is a type of regulation of timing of catagen [GO:0051794]; RO_0002212 catagen [GO:0042637] Sources: GOC:ai, GOC:pr Also known as: inhibition of catagen, down regulation of catagen, down-regulation of catagen, downregulation of catagen, negative regulation of catagen Definition: Any process that stops, prevents, or reduces the frequency, rate or extent of timing of catagen, the regression phase of the hair cycle.